{
  "gene_name": "Metallothionein-1X",
  "term_id": "GO:0071294",
  "term_label": "cellular response to zinc ion",
  "gene": "UniProtKB:P80297",
  "gene_symbol": "MT1X"
}